{
  "gene_name": "Early growth response protein 1",
  "gene_symbol": "EGR1",
  "term_label": "long-term memory",
  "term_id": "GO:0007616",
  "gene": "UniProtKB:P18146"
}